{
  "gene_name": "Zinc finger protein 383",
  "term_id": "GO:0000978",
  "gene_symbol": "ZNF383",
  "gene": "UniProtKB:Q8NA42",
  "term_label": "RNA polymerase II cis-regulatory region sequence-specific DNA binding"
}